{
  "gene_symbol": "C17orf75",
  "gene_name": "Protein Njmu-R1",
  "term_id": "GO:0005802",
  "term_label": "trans-Golgi network",
  "gene": "UniProtKB:Q9HAS0"
}